chitin-based cuticle development [GO:0040003] (biological process) Relationships: is a type of cuticle development [GO:0042335] Sources: GOC:mtg_sensu Subtypes: chitin-based embryonic cuticle biosynthetic process [GO:0008362], adult chitin-based cuticle development [GO:0008365], cuticle development involved in chitin-based cuticle molting cycle [GO:0042337] Definition: Synthesis and deposition of a chitin-based noncellular, hardened, or membranous secretion from an epithelial sheet. An example of this process is found in Drosophila melanogaster. Also known as: chitin-based cuticle anabolism, chitin-based cuticle biosynthetic process, chitin-based cuticle formation, chitin-based cuticle synthesis